histone methacryllysine demethacrylase activity [GO:0140219] (molecular function) References: PMID:34961760 Relationships: is a type of GO:0140993 Definition: Catalysis of the reaction: N6-methacrylyl-L-lysyl-[histone] + H2O = 2-methylprop-2-enoate + L-lysyl-[histone].